beta-galactosidase complex [GO:0009341] (cellular component) Relationships: is_a catalytic complex [GO:1902494] References: PMID:15950161 Definition: A protein complex that possesses beta-galactosidase activity, i.e. catalyzes the hydrolysis of terminal non-reducing beta-D-galactose residues in beta-D-galactosides. In E. coli, the complex is a homotetramer; dimeric and hexameric beta-galactosidase complexes have been observed in other species.